scopoletin glucosyltransferase activity [GO:0050275] (MF) Also known as: SGTase activity, UDP-glucose:scopoletin O-beta-D-glucosyltransferase activity, UDPglucose:scopoletin O-beta-D-glucosyltransferase activity, UDPglucose:scopoletin glucosyltransferase activity, uridine diphosphoglucose-scopoletin glucosyltransferase activity Definition: Catalysis of the reaction: scopoletin + UDP-D-glucose = H+ + scopolin + UDP. Sources: EC:2.4.1.128, RHEA:20453 Relationships: is a type of UDP-glucosyltransferase activity [GO:0035251]